{
  "gene_symbol": "ANXA1",
  "term_label": "phagocytosis",
  "gene": "UniProtKB:P04083",
  "term_id": "GO:0006909",
  "gene_name": "Annexin A1"
}